{
  "gene_symbol": "MVD",
  "term_id": "GO:0004163",
  "term_label": "diphosphomevalonate decarboxylase activity",
  "gene_name": "Diphosphomevalonate decarboxylase",
  "gene": "UniProtKB:P53602"
}